{
  "term_id": "GO:0042391",
  "gene_name": "CHRNA7-FAM7A fusion protein",
  "gene_symbol": "CHRFAM7A",
  "term_label": "regulation of membrane potential",
  "gene": "UniProtKB:Q494W8"
}